nuclear migration by microtubule mediated pushing forces [GO:0098863] (biological process) Relationships: is a type of nuclear migration [GO:0007097]; is a type of GO:0099098; is a type of GO:0099111 Definition: The directed movement of the nucleus by pushing forces exerted by polymerization of backward-extending microtubules. References: PMID:11309419, PMID:16611238 Sources: GOC:vw